oxidoreductase activity, acting on other nitrogenous compounds as donors, with NAD or NADP as acceptor [GO:0046857] (molecular function) Definition: Catalysis of an oxidation-reduction (redox) reaction in which a nitrogenous group, excluding NH and NH2 groups, acts as a hydrogen or electron donor and reduces NAD or NADP. Sources: EC:1.7.1.-, GOC:jl Subtypes: GMP reductase activity [GO:0003920], GO:0008942, nitrobenzene nitroreductase (NADPH) activity [GO:0018546], preQ1 synthase activity [GO:0033739], 4-(dimethylamino)phenylazoxybenzene reductase activity [GO:0047136], N-hydroxy-2-acetamidofluorene reductase [NAD(P)H] activity [GO:0047137], hyponitrite reductase (NADH) activity [GO:0047999], azobenzene reductase (NADP+) activity [GO:0050446], hydroxylamine reductase (NADH) activity [GO:0050460], GO:0050463, nitroquinoline-N-oxide reductase [NAD(P)H] activity [GO:0050465], nitric oxide reductase [NAD(P)H] activity [GO:0102199] Relationships: is a type of oxidoreductase activity, acting on other nitrogenous compounds as donors [GO:0016661]